{
  "gene_symbol": "CSTF3",
  "gene": "UniProtKB:Q12996",
  "term_label": "RNA 3'-end processing",
  "gene_name": "Cleavage stimulation factor subunit 3",
  "term_id": "GO:0031123"
}